{
  "gene_symbol": "ILVBL",
  "gene": "UniProtKB:A1L0T0",
  "term_label": "flavin adenine dinucleotide binding",
  "gene_name": "2-hydroxyacyl-CoA lyase 2",
  "term_id": "GO:0050660"
}